{
  "term_label": "regulation of actin filament polymerization",
  "gene": "UniProtKB:O94868",
  "term_id": "GO:0030833",
  "gene_symbol": "FCHSD2",
  "gene_name": "F-BAR and double SH3 domains protein 2"
}